{
  "gene_name": "Serine palmitoyltransferase 1",
  "term_id": "GO:0046513",
  "term_label": "ceramide biosynthetic process",
  "gene_symbol": "SPTLC1",
  "gene": "UniProtKB:O15269"
}